{
  "gene": "UniProtKB:O60711",
  "term_label": "substrate adhesion-dependent cell spreading",
  "term_id": "GO:0034446",
  "gene_symbol": "LPXN",
  "gene_name": "Leupaxin"
}